hexadecanal dehydrogenase (acylating) activity [GO:0047104] (molecular function) Sources: EC:1.2.1.42, RHEA:19705 Also known as: fatty acyl-CoA reductase activity, hexadecanal:NAD+ oxidoreductase (CoA-acylating) Relationships: is a type of long-chain fatty aldehyde dehydrogenase (NAD+) activity [GO:0050061] Definition: Catalysis of the reaction: CoA + NAD+ + palmitaldehyde = H+ + NADH + palmitoyl-CoA.